{
  "gene": "UniProtKB:O14910",
  "gene_name": "Protein lin-7 homolog A",
  "gene_symbol": "LIN7A",
  "term_id": "GO:0007269",
  "term_label": "neurotransmitter secretion"
}